{
  "term_id": "GO:0000776",
  "gene_symbol": "CKAP5",
  "gene_name": "Cytoskeleton-associated protein 5",
  "gene": "UniProtKB:Q14008",
  "term_label": "kinetochore"
}